extracellular matrix of synaptic cleft [GO:0098965] (cellular component) Relationships: is a type of specialized extracellular matrix [GO:0140047]; is part of GO:0099535 Sources: GOC:dos Also known as: ECM of synaptic cleft, synaptic cleft ECM Definition: The portion of the extracellular matrix that lies within the synaptic cleft.